laricitrin 5'-O-methyltransferase activity [GO:0070448] (molecular function) Sources: RHEA:25633 Relationships: is a type of O-methyltransferase activity [GO:0008171]; is a type of S-adenosylmethionine-dependent methyltransferase activity [GO:0008757] Definition: Catalysis of the reaction: S-adenosyl-L-methionine + laricitrin = S-adenosyl-L-homocysteine + syringetin. Also known as: CrCOMT2, S-adenosyl-L-methionine:myricetin O-methyltransferase activity, flavonoid 3',5'-O-dimethyltransferase activity